{
  "term_id": "UNKNOWN:0002",
  "gene": "UniProtKB:Q9UIF9",
  "gene_symbol": "BAZ2A",
  "term_label": "Unknown biological process",
  "gene_name": "Bromodomain adjacent to zinc finger domain protein 2A"
}